chondrocyte differentiation involved in endochondral bone morphogenesis [GO:0003413] (biological process) Relationships: is a type of GO:0002062; is part of cartilage development involved in endochondral bone morphogenesis [GO:0060351] Subtypes: growth plate cartilage chondrocyte differentiation [GO:0003418] Regulation: regulated by regulation of chondrocyte differentiation involved in endochondral bone morphogenesis [GO:1902738] Definition: The process in which a chondroblast acquires specialized structural and/or functional features of a chondrocyte that will contribute to the development of a bone. A chondrocyte is a polymorphic cell that forms cartilage. Sources: GOC:ascb_2009, GOC:dph, GOC:tb